{
  "gene": "UniProtKB:A2VDJ0",
  "gene_name": "Transmembrane protein 131-like",
  "term_label": "negative regulation of canonical Wnt signaling pathway",
  "term_id": "GO:0090090",
  "gene_symbol": "TMEM131L"
}